postsynaptic density protein 95 clustering [GO:0097119] (biological process) Definition: The clustering process in which postsynaptic density protein 95 (PSD-95) molecules are localized to distinct domains in the cell membrane. PSD-95 is mostly located in the post synaptic density of neurons, and is involved in anchoring synaptic proteins. References: PMID:10433269 Sources: GOC:BHF, GOC:sjp Also known as: Dlg4 clustering, PSD-95 clustering, post-synaptic density protein 95 clustering Relationships: is a type of protein localization to membrane [GO:0072657]; BFO_0000050 GO:0001941; is part of GO:0097106 Regulation: regulated by regulation of postsynaptic density protein 95 clustering [GO:1902897]